negative regulation of cellular response to caffeine [GO:1901181] (biological process) Sources: GOC:TermGenie Definition: Any process that stops, prevents or reduces the frequency, rate or extent of cellular response to caffeine. Also known as: down regulation of cellular response to caffeine, down-regulation of cellular response to caffeine, downregulation of cellular response to caffeine, inhibition of cellular response to caffeine Relationships: is a type of GO:0048523; is a type of negative regulation of response to stimulus [GO:0048585]; negatively regulates cellular response to caffeine [GO:0071313]